negative adaptation of signaling pathway [GO:0022401] (biological process) Sources: GOC:isa_complete Also known as: negative adaptation of signal transduction pathway, negative adaptation of signalling pathway Definition: The negative regulation of a signal transduction pathway in response to a stimulus upon prolonged exposure to that stimulus. Relationships: is a type of negative regulation of signal transduction [GO:0009968]; is a type of GO:0023058 Subtypes: adaptation to pheromone regulating conjugation with mutual genetic exchange [GO:0000760], negative adaptation of signaling pathway by response to pheromone involved in pheromone-induced unidirectional conjugation [GO:0000766], GO:0002029